{
  "gene_symbol": "KCNMB4",
  "gene": "UniProtKB:Q86W47",
  "term_id": "GO:0005513",
  "term_label": "detection of calcium ion",
  "gene_name": "Calcium-activated potassium channel subunit beta-4"
}